fruit abscission [GO:0060867] (biological process) Definition: The controlled shedding of a fruit. Sources: GOC:dph, GOC:sdb_2009, GOC:tb Relationships: is a type of abscission [GO:0009838]